{
  "gene": "UniProtKB:Q5VT40",
  "term_id": "UNKNOWN:0001",
  "gene_symbol": "FAM78B",
  "gene_name": "Protein FAM78B",
  "term_label": "Unknown molecular function"
}